{
  "term_label": "3'-UTR-mediated mRNA destabilization",
  "gene_name": "Endoribonuclease ZC3H12A",
  "gene": "UniProtKB:Q5D1E8",
  "term_id": "GO:0061158",
  "gene_symbol": "ZC3H12A"
}